{
  "gene": "UniProtKB:Q9BY42",
  "term_id": "UNKNOWN:0002",
  "gene_symbol": "RTF2",
  "gene_name": "Replication termination factor 2",
  "term_label": "Unknown biological process"
}